{
  "term_label": "Unknown molecular function",
  "gene": "UniProtKB:Q9HBF5",
  "gene_name": "Suppressor of tumorigenicity 20 protein",
  "gene_symbol": "ST20",
  "term_id": "UNKNOWN:0001"
}